{
  "gene": "UniProtKB:P39023",
  "term_label": "cytosolic large ribosomal subunit",
  "gene_name": "Large ribosomal subunit protein uL3",
  "gene_symbol": "RPL3",
  "term_id": "GO:0022625"
}